cobalamin transport complex [GO:1990191] (cellular component) References: PMID:22569249 Sources: GOC:bhm Also known as: BtuCDF complex, cobalamin-transporting BtuCDF complex, vitamin B12 transport complex, vitamin B12-transporting BtuCDF complex Relationships: is a type of ATP-binding cassette (ABC) transporter complex [GO:0043190]; has part BtuCD complex [GO:1990193] Definition: Protein complex facilitating ATP-dependent cobalamin (vitamin B12) transport through inner cell membrane (periplasm to cytoplasm) in Gram-negative bacteria. In E. coli the system is composed of a periplasmic cobalamin-binding protein (BtuF), an integral membrane homodimer, BtuC, and a cytoplasmic ATP-binding homodimer BtuD.